{
  "term_label": "methylation",
  "gene_name": "Acetylserotonin O-methyltransferase",
  "term_id": "GO:0032259",
  "gene_symbol": "ASMT",
  "gene": "UniProtKB:P46597"
}